{
  "gene_name": "Early growth response protein 4",
  "term_id": "GO:0000978",
  "term_label": "RNA polymerase II cis-regulatory region sequence-specific DNA binding",
  "gene": "UniProtKB:Q05215",
  "gene_symbol": "EGR4"
}